{
  "term_id": "GO:0050807",
  "gene": "UniProtKB:Q8WZ74",
  "gene_name": "Cortactin-binding protein 2",
  "term_label": "regulation of synapse organization",
  "gene_symbol": "CTTNBP2"
}